{
  "gene_symbol": "ARHGAP4",
  "term_label": "negative regulation of cell migration",
  "gene_name": "Rho GTPase-activating protein 4",
  "gene": "UniProtKB:P98171",
  "term_id": "GO:0030336"
}